inositol phosphoceramide synthase regulator activity [GO:0070917] (molecular function) Relationships: is a type of enzyme regulator activity [GO:0030234]; regulates inositol phosphoceramide synthase activity [GO:0045140] Definition: Binds to and modulates the activity of inositol phosphoceramide synthase. Sources: GOC:mah Note: See also the molecular function term 'histone acetyltransferase activity ; GO:0004402'. Also known as: IPC synthase regulator activity